dihydropterin deaminase activity [GO:0004153] (molecular function) Relationships: is a type of hydrolase activity, acting on carbon-nitrogen (but not peptide) bonds, in cyclic amidines [GO:0016814]; is a type of deaminase activity [GO:0019239] References: PMID:19567870, PMID:38786926 Sources: GOC:jl Definition: Catalysis of the reaction: 7,8-dihydropterin + H2O = 7,8-dihydrolumazine + NH3.